{
  "term_label": "Unknown biological process",
  "gene_symbol": "TYMSOS",
  "gene_name": "TYMS opposite strand protein",
  "term_id": "UNKNOWN:0002",
  "gene": "UniProtKB:Q8TAI1"
}